oxidative RNA demethylation [GO:0035513] (biological process) References: PMID:12594517, PMID:16482161, PMID:18775698 Definition: The removal of the methyl group from one or more nucleotides within an RNA molecule involving oxidation (i.e. electron loss) of one or more atoms. Relationships: is a type of RNA modification [GO:0009451]; is a type of oxidative demethylation [GO:0070989]